{
  "gene": "UniProtKB:Q9ULP9",
  "gene_symbol": "TBC1D24",
  "term_label": "Unknown molecular function",
  "term_id": "UNKNOWN:0001",
  "gene_name": "TBC1 domain family member 24"
}